{
  "term_label": "G protein-coupled receptor signaling pathway",
  "term_id": "GO:0007186",
  "gene_name": "Trace amine-associated receptor 8",
  "gene": "UniProtKB:Q969N4",
  "gene_symbol": "TAAR8"
}